{
  "gene_name": "Immunoglobulin-like domain-containing receptor 2",
  "gene": "UniProtKB:Q71H61",
  "term_id": "GO:0031016",
  "gene_symbol": "ILDR2",
  "term_label": "pancreas development"
}